negative regulation of programmed cell death [GO:0043069] (biological process) Also known as: down regulation of programmed cell death, down-regulation of programmed cell death, downregulation of programmed cell death, inhibition of programmed cell death, negative regulation of non-apoptotic programmed cell death Sources: GOC:jl Definition: Any process that stops, prevents, or reduces the frequency, rate or extent of programmed cell death, cell death resulting from activation of endogenous cellular processes. Relationships: is a type of regulation of programmed cell death [GO:0043067]; is a type of negative regulation of cellular process [GO:0048523]; negatively regulates programmed cell death [GO:0012501] Subtypes: negative regulation of plant-type hypersensitive response [GO:0034051], negative regulation of apoptotic process [GO:0043066], negative regulation of retinal cell programmed cell death [GO:0046671], GO:0062099, negative regulation of ferroptosis [GO:0110076], GO:1901299, negative regulation of autophagic cell death [GO:1904093], GO:1905716